phosphoribosylamine-glycine ligase activity [GO:0004637] (molecular function) Also known as: 2-amino-N-ribosylacetamide 5'-phosphate kinosynthase activity, 5'-phosphoribosylglycinamide synthetase activity, 5-phospho-D-ribosylamine:glycine ligase (ADP-forming), GAR, GAR synthetase activity, GARS activity, glycinamide ribonucleotide synthetase activity, glycineamide ribonucleotide synthetase activity, phosphoribosylglycinamide synthetase activity, phosphoribosylglycineamide synthetase activity Definition: Catalysis of the reaction: 5-phospho-D-ribosylamine + ATP + glycine = N(1)-(5-phospho-D-ribosyl)glycinamide + ADP + 2 H+ + phosphate. Relationships: is a type of ligase activity, forming carbon-nitrogen bonds [GO:0016879] Sources: EC:6.3.4.13, RHEA:17453